negative regulation of triglyceride storage [GO:0010891] (biological process) Relationships: is a type of GO:0010888; is a type of GO:0010889; negatively regulates triglyceride storage [GO:0030730] Also known as: negative regulation of sequestering of triacylglycerol, negative regulation of sequestering of triglyceride, negative regulation of triglyceride sequestration Definition: Any process that decreases the rate, frequency or extent of sequestering of triglyceride. Triglyceride sequestration is the process of binding or confining any triester of glycerol such that it is separated from other components of a biological system. Sources: GOC:BHF, GOC:dph, GOC:tb